polymeric immunoglobulin binding [GO:0001790] (MF) Sources: GOC:add, ISBN:0781735149 Relationships: is_a immunoglobulin binding [GO:0019865] Definition: Binding to a J-chain-containing polymeric immunoglobulin of the IgA or IgM isotypes.